{
  "term_id": "GO:0000786",
  "term_label": "nucleosome",
  "gene_symbol": "H2AP",
  "gene": "UniProtKB:O75409",
  "gene_name": "Huntingtin-interacting protein M"
}